positive regulation of smoothened signaling pathway [GO:0045880] (biological process) Definition: Any process that activates or increases the frequency, rate or extent of smoothened signaling. Relationships: is a type of regulation of smoothened signaling pathway [GO:0008589]; is a type of GO:0009967; positively regulates GO:0007224 Sources: GOC:go_curators Also known as: positive regulation of hedgehog signaling pathway, positive regulation of hh signaling pathway, positive regulation of smoothened signalling pathway, up regulation of smoothened signaling pathway, up-regulation of smoothened signaling pathway, upregulation of smoothened signaling pathway, activation of smoothened signaling pathway, stimulation of smoothened signaling pathway, positive regulation of smoothened by patched, positive regulation of smoothened receptor activity by patched Subtypes: GO:1901622